ent-kaurene oxidation to kaurenoic acid [GO:0010241] (biological process) Definition: The three successive oxidations of the 4-methyl group of ent-kaurene to form ent-kaur-16-en-19-oate, kaurenoic acid. This process may be carried out entirely by the enzyme ent-kaurene oxidase. Sources: GOC:tb Also known as: ent-kaurene oxidation to ent-kaur-16-en-19-oate, ent-kaurene oxidation to ent-kaurenoate, ent-kaurene oxidation to kaurenoic acid by ent-kaurene oxidase Note: Note that this term was in molecular function but was moved to biological process as it represents three successive reactions. Relationships: is a type of ent-kaurene metabolic process [GO:0033331]; has part ent-kaurene oxidase activity [GO:0052615]